{
  "gene": "UniProtKB:P16435",
  "term_label": "FMN binding",
  "gene_symbol": "POR",
  "gene_name": "NADPH--cytochrome P450 reductase",
  "term_id": "GO:0010181"
}